{
  "gene_name": "Keratin-associated protein 2-2",
  "gene_symbol": "KRTAP2-2",
  "gene": "UniProtKB:Q9BYT5",
  "term_id": "UNKNOWN:0003",
  "term_label": "Unknown cellular component"
}